very long-chain fatty acid omega-hydroxylase activity [GO:0140692] (molecular function) Definition: Catalysis of the reaction: an omega-methyl-very-long-chain fatty acid + O2 + reduced [NADPH-hemoprotein reductase] = an omega-hydroxy-very-long-chain fatty acid + H+ + H2O + oxidized [NADPH-hemoprotein reductase]. A very long-chain fatty acid has an aliphatic tail containing more than 22 carbons. References: PMID:16547005 Sources: RHEA:67952 Relationships: is a type of fatty acid omega-hydroxylase activity [GO:0120250] Note: While there is not universal consensus on the lengths of short-, medium-, long- and very-long-chain fatty acids, the GO uses the definitions in ChEBI (see CHEBI:26666, CHEBI:59554, CHEBI:15904 and CHEBI:27283).